endocardium development [GO:0003157] (biological process) Relationships: is a type of anatomical structure development [GO:0048856]; is part of heart development [GO:0007507] Definition: The process whose specific outcome is the progression of the endocardium over time, from its formation to the mature structure. The endocardium is an anatomical structure comprised of an endothelium and an extracellular matrix that forms the innermost layer of tissue of the heart, and lines the heart chambers. Sources: GOC:mtg_heart